trans-synaptic signaling via exosome [GO:0099157] (biological process) Also known as: exosome mediated transynaptic signalling, trans-synaptic signalling via exosome References: PMID:19837038 Sources: GOC:dos Relationships: is a type of cell-cell signaling via exosome [GO:0099156]; is a type of GO:0099537 Definition: Transynaptic signaling in which the ligand is carried across the synapse by an exosome.